sulfopyruvate decarboxylase complex [GO:0044681] (cellular component) Relationships: is a type of catalytic complex [GO:1902494] Definition: A complex of two polypeptides which form a dodecamer (A6B6). Catalyzes the decarboxylation of sulfopyruvic acid to sulfoacetaldehyde. This reaction is involved in coenzyme M biosynthesis. References: PMID:10940029 Sources: GOC:mengo_curators